{
  "gene_symbol": "ENAH",
  "term_label": "plasma membrane",
  "gene": "UniProtKB:Q8N8S7",
  "term_id": "GO:0005886",
  "gene_name": "Protein enabled homolog"
}